insect visual primordium formation [GO:0001744] (biological process) Relationships: is a type of GO:0060788; is part of insect visual primordium development [GO:0001748] Definition: Establishment of the optic lobe placode. In Drosophila, for example, the placode appears in the dorsolateral region of the head in late stage 11 embryos and is the precursor to the larval visual system. Also known as: optic lobe and Bolwig's organ precursor formation, optic lobe placode formation References: PMID:8402833 Sources: GOC:mtg_sensu